host organelle outer membrane [GO:0039661] (CC) Subtypes: host cell mitochondrial outer membrane [GO:0044193], host cell nuclear outer membrane [GO:0044202] Sources: GOC:bf, GOC:ch Relationships: is a type of host outer membrane [GO:0044384] Definition: The outer, i.e. cytoplasm-facing in a cellular organelle, lipid bilayer of an organelle envelope, occurring in a host cell.